negative regulation of double-strand break repair via break-induced replication [GO:1901592] (biological process) Relationships: is a type of GO:1901591; is a type of negative regulation of double-strand break repair via homologous recombination [GO:2000042]; negatively regulates double-strand break repair via break-induced replication [GO:0000727] Definition: Any process that stops, prevents or reduces the frequency, rate or extent of double-strand break repair via break-induced replication. Sources: GOC:TermGenie Also known as: down regulation of double-strand break repair via break-induced replication, down-regulation of double-strand break repair via break-induced replication, downregulation of double-strand break repair via break-induced replication, inhibition of double-strand break repair via break-induced replication